intracellularly cGMP-activated cation channel activity [GO:0005223] (molecular function) Definition: Enables the transmembrane transfer of a cation by a channel that opens when intracellular cGMP has been bound by the channel complex or one of its constituent parts. Sources: GOC:mtg_transport Also known as: intracellular cGMP activated cation channel activity, intracellular cGMP-activated cation channel activity Relationships: is a type of intracellularly cyclic nucleotide-activated monoatomic cation channel activity [GO:0005221]